integrator complex [GO:0032039] (cellular component) Definition: A protein complex that stably associates with the C-terminus of RNA polymerase II and mediates 3'-end processing of small nuclear RNAs generated by RNA polymerase II. References: PMID:16239144 Relationships: is a type of GO:0140513